N(1)-acetylpolyamine oxidase (3-acetamidopropanal-forming) activity [GO:0052903] (molecular function) Relationships: is a type of polyamine oxidase activity [GO:0046592] Definition: Catalysis of the reaction: H2O + N(1)-acetylspermine + O2 = 3-acetamidopropanal + H2O2 + spermidine. Also converts N(1)-acetylspermidine to putrescine. Also known as: N(1)-acetylpolyamine oxidase activity, N1-acetylspermidine:oxygen oxidoreductase (3-acetamidopropanal-forming) activity, N1-acetylspermine:oxygen oxidoreductase (3-acetamidopropanal-forming) activity Sources: EC:1.5.3.13